neuron intrinsic apoptotic signaling pathway in response to hydrogen peroxide [GO:0036482] (biological process) Regulation: regulated by regulation of hydrogen peroxide-induced neuron intrinsic apoptotic signaling pathway [GO:1903383]; negatively regulated by negative regulation of hydrogen peroxide-induced neuron intrinsic apoptotic signaling pathway [GO:1903384] Sources: GOC:PARL, GOC:bf Definition: The series of molecular signals in which an intracellular signal is conveyed to trigger the apoptotic death of a neuron in response to hydrogen peroxide. Also known as: hydrogen peroxide-induced neuron apoptosis, hydrogen peroxide-induced neuronal apoptosis, H2O2-induced neuron intrinsic apoptotic signaling pathway, neuron intrinsic apoptotic signaling pathway in response to H2O2, neuron apoptosis in response to hydrogen peroxide Relationships: is a type of neuron intrinsic apoptotic signaling pathway in response to oxidative stress [GO:0036480]; is a type of GO:0036481